{
  "term_id": "GO:0042470",
  "gene": "UniProtKB:O00194",
  "term_label": "melanosome",
  "gene_symbol": "RAB27B",
  "gene_name": "Ras-related protein Rab-27B"
}